geranylfarnesyl diphosphate synthase activity [GO:0044687] (molecular function) References: PMID:20097171 Sources: RHEA:25694 Relationships: is a type of prenyl diphosphate synthase activity [GO:0120531] Also known as: FGPP synthase activity Definition: Catalysis of the reaction: (2E,6E,10E)-geranylgeranyl diphosphate + isopentenyl diphosphate = (2E,6E,10E,14E)-geranylfarnesyl diphosphate + diphosphate.